{
  "gene_name": "Telomere length regulation protein TEL2 homolog",
  "gene": "UniProtKB:Q9Y4R8",
  "gene_symbol": "TELO2",
  "term_label": "Hsp90 protein binding",
  "term_id": "GO:0051879"
}